helvolic acid biosynthetic process [GO:1900812] (biological process) Definition: The chemical reactions and pathways resulting in the formation of helvolic acid. Sources: GOC:TermGenie, GOC:di Relationships: is a type of steroid biosynthetic process [GO:0006694]; is a type of ketone biosynthetic process [GO:0042181]; is a type of secondary metabolite biosynthetic process [GO:0044550]; is a type of carboxylic acid biosynthetic process [GO:0046394]; is a type of olefinic compound biosynthetic process [GO:0120255] Regulation: regulated by regulation of helvolic acid biosynthetic process [GO:1900840]; negatively regulated by negative regulation of helvolic acid biosynthetic process [GO:1900841]; positively regulated by positive regulation of helvolic acid biosynthetic process [GO:1900842] Also known as: helvolic acid anabolism, helvolic acid biosynthesis, helvolic acid formation, helvolic acid synthesis, Fumigacin anabolism, Fumigacin biosynthesis, Fumigacin biosynthetic process, Fumigacin formation, Fumigacin synthesis